{
  "gene": "UniProtKB:Q13258",
  "term_id": "GO:0005886",
  "gene_symbol": "PTGDR",
  "term_label": "plasma membrane",
  "gene_name": "Prostaglandin D2 receptor"
}